diapedesis [GO:0050904] (biological process) Definition: The passage of a leukocyte between the tight junctions of endothelial cells lining blood vessels, typically the fourth and final step of cellular extravasation. References: PMID:14680625, PMID:14708592, PMID:7507411, PMID:8600538 Sources: ISBN:0781735149 Relationships: is_a leukocyte migration [GO:0050900]; is part of cellular extravasation [GO:0045123] Subtypes: helper T cell diapedesis [GO:0035685] Note: Note that the term diapedesis, although sometimes used as a direct synonym for cellular extravasation, is used here for the specific final step of the process, in concordance with recent reviews of the topic.